{
  "gene_symbol": "CD46",
  "term_id": "GO:0005886",
  "term_label": "plasma membrane",
  "gene_name": "Membrane cofactor protein",
  "gene": "UniProtKB:P15529"
}